{
  "term_label": "regulation of transcription by RNA polymerase II",
  "term_id": "GO:0006357",
  "gene_symbol": "ZNF705A",
  "gene": "UniProtKB:Q6ZN79",
  "gene_name": "Zinc finger protein 705A"
}